{
  "gene": "UniProtKB:Q8WXQ3",
  "gene_symbol": "LINC01599",
  "term_id": "UNKNOWN:0002",
  "gene_name": "Putative uncharacterized protein encoded by LINC01599",
  "term_label": "Unknown biological process"
}